{
  "term_label": "Unknown cellular component",
  "term_id": "UNKNOWN:0003",
  "gene": "UniProtKB:Q5I0G3",
  "gene_name": "Putative malate dehydrogenase 1B",
  "gene_symbol": "MDH1B"
}